{
  "gene": "UniProtKB:P25788",
  "term_id": "GO:0043161",
  "gene_name": "Proteasome subunit alpha type-3",
  "term_label": "proteasome-mediated ubiquitin-dependent protein catabolic process",
  "gene_symbol": "PSMA3"
}